{
  "gene_name": "Putative uncharacterized protein PRO1854",
  "gene": "UniProtKB:Q9UHT4",
  "term_id": "UNKNOWN:0001",
  "gene_symbol": "PRO1854",
  "term_label": "Unknown molecular function"
}